{
  "gene": "UniProtKB:O00222",
  "gene_symbol": "GRM8",
  "term_id": "GO:0001642",
  "term_label": "group III metabotropic glutamate receptor activity",
  "gene_name": "Metabotropic glutamate receptor 8"
}